3-hydroxyanthranilate oxidase activity [GO:0047561] (molecular function) Relationships: is a type of oxidoreductase activity, acting on diphenols and related substances as donors, oxygen as acceptor [GO:0016682] Also known as: 3-hydroxyanthranilate:oxygen oxidoreductase activity, 3-hydroxyanthranilic acid oxidase activity Sources: EC:1.10.3.5, RHEA:17245 Definition: Catalysis of the reaction: 3-hydroxyanthranilate + O2 = 6-imino-5-oxocyclohexa-1,3-dienecarboxylate + H2O2.